{
  "gene_name": "Small cysteine and glycine repeat-containing protein 5",
  "gene_symbol": "SCYGR5",
  "gene": "UniProtKB:A0A286YF46",
  "term_id": "UNKNOWN:0003",
  "term_label": "Unknown cellular component"
}